{
  "gene_symbol": "MAP4K4",
  "term_label": "cytoplasm",
  "gene": "UniProtKB:O95819",
  "term_id": "GO:0005737",
  "gene_name": "Mitogen-activated protein kinase kinase kinase kinase 4"
}